{
  "gene_symbol": "DOCK1",
  "gene_name": "Dedicator of cytokinesis protein 1",
  "term_label": "myoblast fusion",
  "term_id": "GO:0007520",
  "gene": "UniProtKB:Q14185"
}